centriolar satellite [GO:0034451] (cellular component) References: PMID:10579718, PMID:12403812 Sources: GOC:BHF Definition: A small (70-100 nm) cytoplasmic granule that contains a number of centrosomal proteins; centriolar satellites traffic toward microtubule minus ends and are enriched near the centrosome. Relationships: is a type of GO:0110165; is part of centrosome [GO:0005813]